dGDP binding [GO:0032566] (molecular function) Definition: Binding to dGDP, deoxyguanosine diphosphate. Relationships: is a type of GO:0032560; is a type of anion binding [GO:0043168] Sources: GOC:mah